negative regulation of blood coagulation, intrinsic pathway [GO:2000267] (biological process) Definition: Any process that stops, prevents or reduces the frequency, rate or extent of blood coagulation, intrinsic pathway. Sources: GOC:mah Relationships: is a type of GO:0030195; is_a GO:2000258; is a type of regulation of blood coagulation, intrinsic pathway [GO:2000266]; negatively regulates GO:0007597